{
  "gene_name": "cAMP-dependent protein kinase type II-beta regulatory subunit",
  "term_id": "GO:0004862",
  "gene_symbol": "PRKAR2B",
  "gene": "UniProtKB:P31323",
  "term_label": "cAMP-dependent protein kinase inhibitor activity"
}